histone H4K20 methyltransferase activity [GO:0042799] (molecular function) Relationships: is a type of protein-lysine N-methyltransferase activity [GO:0016279]; is a type of histone H4 methyltransferase activity [GO:0140939] Definition: Catalysis of the reaction: S-adenosyl-L-methionine + histone H4 L-lysine (position 20) = S-adenosyl-L-homocysteine + histone H4 N6-methyl-L-lysine (position 20). This reaction is the addition of a methyl group to the lysine residue at position 20 of the histone H4 protein. Subtypes: histone H4K20me methyltransferase activity [GO:0140941], histone H4K20 trimethyltransferase activity [GO:0140943], histone H4K20 monomethyltransferase activity [GO:0140944] References: PMID:12086618 Note: Note that the residue position corresponds to the canonical human H4 histone (UniProtKB:P02309); this residue is conserved across all eukaryotes. Note that the initiation methionine is cleaved, so the first residue is S1. Also known as: histone H4K20 methylase activity, histone H4 lysine 20-specific methyltransferase activity, histone H4K20 methylation, histone lysine N-methyltransferase activity (H4-K20 specific), histone methylase activity (H4-K20 specific), histone methyltransferase activity (H4-K20 specific), histone-H4K20 methyltransferase activity